{
  "term_id": "GO:0001579",
  "gene": "UniProtKB:Q6P1M0",
  "gene_name": "Long-chain fatty acid transport protein 4",
  "gene_symbol": "SLC27A4",
  "term_label": "medium-chain fatty acid transport"
}